{
  "term_id": "GO:0001523",
  "gene_name": "Short-chain dehydrogenase_reductase 3",
  "term_label": "retinoid metabolic process",
  "gene": "UniProtKB:O75911",
  "gene_symbol": "DHRS3"
}